{
  "term_label": "DNA-binding transcription factor activity, RNA polymerase II-specific",
  "term_id": "GO:0000981",
  "gene_symbol": "ZNF730",
  "gene": "UniProtKB:Q6ZMV8",
  "gene_name": "Putative zinc finger protein 730"
}